{
  "gene": "UniProtKB:Q53H54",
  "gene_name": "tRNA wybutosine-synthesizing protein 2 homolog",
  "gene_symbol": "TRMT12",
  "term_id": "GO:0008175",
  "term_label": "tRNA methyltransferase activity"
}